positive regulation of cell development [GO:0010720] (biological process) Sources: GOC:BHF, GOC:dph, GOC:tb Relationships: is a type of positive regulation of cell differentiation [GO:0045597]; is a type of GO:0060284; positively regulates cell development [GO:0048468] Subtypes: GO:0010770, positive regulation of eye photoreceptor cell development [GO:0042479], GO:0048743, positive regulation of neurogenesis [GO:0050769], positive regulation of cardiac muscle fiber development [GO:0055020], positive regulation of oocyte development [GO:0060282], positive regulation of metula development [GO:0070804], positive regulation of phialide development [GO:0070807], positive regulation of Hulle cell development [GO:0070810], positive regulation of spore encystment on host [GO:0075216], positive regulation of ascospore formation [GO:0075296], positive regulation of conidium formation [GO:0075307], positive regulation of establishment of blood-brain barrier [GO:0090211], positive regulation of endothelial cell development [GO:1901552], positive regulation of chondrocyte development [GO:1902761], positive regulation of cell maturation [GO:1903431], positive regulation of hemopoiesis [GO:1903708], positive regulation of establishment of Sertoli cell barrier [GO:1904446], GO:1905081, positive regulation of intestinal epithelial cell development [GO:1905300], positive regulation of oogenesis [GO:1905881], positive regulation of type B pancreatic cell development [GO:2000078], positive regulation of metanephric podocyte development [GO:2000478] Definition: Any process that increases the rate, frequency or extent of the progression of the cell over time, from its formation to the mature structure. Cell development does not include the steps involved in committing a cell to a specific fate.